{
  "gene_symbol": "NFATC4",
  "term_id": "GO:0000981",
  "term_label": "DNA-binding transcription factor activity, RNA polymerase II-specific",
  "gene_name": "Nuclear factor of activated T-cells, cytoplasmic 4",
  "gene": "UniProtKB:Q14934"
}